{
  "gene": "UniProtKB:Q92523",
  "gene_name": "Carnitine O-palmitoyltransferase 1, muscle isoform",
  "term_id": "GO:0009437",
  "gene_symbol": "CPT1B",
  "term_label": "carnitine metabolic process"
}